{
  "term_label": "nucleus",
  "gene": "UniProtKB:Q02363",
  "gene_symbol": "ID2",
  "term_id": "GO:0005634",
  "gene_name": "DNA-binding protein inhibitor ID-2"
}